{
  "gene_name": "Kalirin",
  "gene": "UniProtKB:O60229",
  "term_label": "axon guidance",
  "gene_symbol": "KALRN",
  "term_id": "GO:0007411"
}